{
  "gene_name": "Proton-coupled zinc antiporter SLC30A8",
  "term_label": "response to zinc ion",
  "term_id": "GO:0010043",
  "gene_symbol": "SLC30A8",
  "gene": "UniProtKB:Q8IWU4"
}